{
  "term_id": "GO:0006303",
  "gene_name": "DNA nucleotidylexotransferase",
  "term_label": "double-strand break repair via nonhomologous end joining",
  "gene": "UniProtKB:P04053",
  "gene_symbol": "DNTT"
}